{
  "gene": "UniProtKB:Q969G5",
  "term_label": "cytoplasm",
  "gene_symbol": "CAVIN3",
  "gene_name": "Caveolae-associated protein 3",
  "term_id": "GO:0005737"
}